{
  "gene": "UniProtKB:Q9Y5F2",
  "term_label": "plasma membrane",
  "gene_name": "Protocadherin beta-11",
  "gene_symbol": "PCDHB11",
  "term_id": "GO:0005886"
}